VAMP4-syntaxin-6-syntaxin-16-Vti1a complex [GO:0070068] (cellular component) Definition: A SNARE complex that contains VAMP4, syntaxin 6, syntaxin 16, and Vti1a (or orthologs thereof). Relationships: is a type of SNARE complex [GO:0031201] References: PMID:11839770 Also known as: SNARE complex (Vamp4, Stx6, Stx16, Vti1a), Vamp4-Stx6-Stx16-Vti1a complex